{
  "term_label": "detection of chemical stimulus involved in sensory perception of smell",
  "gene": "UniProtKB:Q8NGT2",
  "gene_name": "Olfactory receptor 13J1",
  "term_id": "GO:0050911",
  "gene_symbol": "OR13J1"
}